{
  "gene_symbol": "FOXB1",
  "term_id": "UNKNOWN:0003",
  "term_label": "Unknown cellular component",
  "gene_name": "Forkhead box protein B1",
  "gene": "UniProtKB:Q99853"
}